{
  "gene_name": "Leukocyte immunoglobulin-like receptor subfamily B member 2",
  "term_id": "GO:0032396",
  "gene": "UniProtKB:Q8N423",
  "gene_symbol": "LILRB2",
  "term_label": "inhibitory MHC class I receptor activity"
}